{
  "term_label": "glucosyltransferase activity",
  "gene_name": "Protein O-glucosyltransferase 2",
  "gene_symbol": "POGLUT2",
  "term_id": "GO:0046527",
  "gene": "UniProtKB:Q6UW63"
}